{
  "gene_symbol": "HARS1",
  "gene": "UniProtKB:P12081",
  "term_label": "histidine-tRNA ligase activity",
  "gene_name": "Histidine--tRNA ligase, cytoplasmic",
  "term_id": "GO:0004821"
}